{
  "gene_symbol": "NR1H3",
  "term_id": "GO:0030522",
  "term_label": "intracellular receptor signaling pathway",
  "gene": "UniProtKB:Q13133",
  "gene_name": "Oxysterols receptor LXR-alpha"
}